regulation of cellotriose transport [GO:1900285] (biological process) Relationships: is a type of regulation of transport [GO:0051049]; RO_0002211 cellotriose transport [GO:2001096] Sources: GOC:TermGenie, GOC:mengo_curators Definition: Any process that modulates the frequency, rate or extent of cellotriose transport. Subtypes: negative regulation of cellotriose transport [GO:1900286], GO:1900287